{
  "gene_symbol": "NAPSA",
  "term_label": "aspartic-type endopeptidase activity",
  "term_id": "GO:0004190",
  "gene_name": "Napsin-A",
  "gene": "UniProtKB:O96009"
}